cleistothecium development [GO:0070791] (biological process) Relationships: is a type of sporocarp development involved in sexual reproduction [GO:0000909] References: PMID:17446882 Sources: ISBN:0471522295 Regulation: regulated by regulation of cleistothecium development [GO:0070796]; negatively regulated by negative regulation of cleistothecium development [GO:0070797]; RO_0002213 by positive regulation of cleistothecium development [GO:0070798] Definition: The process whose specific outcome is the progression of the cleistothecium over time, from its formation to the mature structure. The cleistothecium is a closed sexual fruiting body that contains ascospores in linear asci, characteristic of some filamentous Ascomycete fungi such as members of the genera Aspergillus and Emericella.